{
  "term_id": "GO:0005694",
  "gene_name": "Protein SPO16 homolog",
  "term_label": "chromosome",
  "gene": "UniProtKB:Q5VVC0",
  "gene_symbol": "SPO16"
}